{
  "gene_symbol": "CD300A",
  "term_id": "GO:0005886",
  "term_label": "plasma membrane",
  "gene_name": "CMRF35-like molecule 8",
  "gene": "UniProtKB:Q9UGN4"
}